{
  "term_label": "cytoplasmic vesicle",
  "gene_symbol": "GBP4",
  "gene": "UniProtKB:Q96PP9",
  "term_id": "GO:0031410",
  "gene_name": "Guanylate-binding protein 4"
}